{
  "gene_name": "Homeobox protein Hox-C10",
  "term_label": "RNA polymerase II cis-regulatory region sequence-specific DNA binding",
  "gene_symbol": "HOXC10",
  "term_id": "GO:0000978",
  "gene": "UniProtKB:Q9NYD6"
}